{
  "gene": "UniProtKB:Q9Y2C9",
  "term_label": "Toll-like receptor 2-Toll-like receptor 6 protein complex",
  "gene_symbol": "TLR6",
  "gene_name": "Toll-like receptor 6",
  "term_id": "GO:0035355"
}